{
  "term_label": "Unknown cellular component",
  "gene": "UniProtKB:Q8IYS1",
  "gene_symbol": "PM20D2",
  "term_id": "UNKNOWN:0003",
  "gene_name": "Xaa-Arg dipeptidase"
}